{
  "gene_name": "Zinc finger CCCH domain-containing protein 4",
  "term_label": "nucleoplasm",
  "term_id": "GO:0005654",
  "gene": "UniProtKB:Q9UPT8",
  "gene_symbol": "ZC3H4"
}